{
  "gene_symbol": "H1-10",
  "term_label": "nucleus",
  "gene": "UniProtKB:Q92522",
  "term_id": "GO:0005634",
  "gene_name": "Histone H1.10"
}